modified amino acid transmembrane transporter activity [GO:0072349] (molecular function) Sources: GOC:mah Definition: Enables the transfer of modified amino acids from one side of a membrane to the other. Subtypes: S-methylmethionine transmembrane transporter activity [GO:0000100], GO:0000514, creatine transmembrane transporter activity [GO:0005308], GO:0008517, GO:0015184, amino-acid betaine transmembrane transporter activity [GO:0015199], GO:0015226, 5-formyltetrahydrofolate transmembrane transporter activity [GO:0015231], GO:0015233, GO:0015327, GO:0015498, GO:0015558, GO:0034590, GO:0034634, GO:0180003, 4-(trimethylammonio)butanoate transmembrane transporter activity [GO:1901236], carcinine transmembrane transporter activity [GO:1905131] Also known as: modified amino acid transporter activity, amino acid derivative transmembrane transporter activity Relationships: is a type of transmembrane transporter activity [GO:0022857]; is part of modified amino acid transport [GO:0072337]